teliospore formation [GO:0075255] (biological process) Regulation: regulated by regulation of teliospore formation [GO:0075256]; RO_0002213 by positive regulation of teliospore formation [GO:0075257]; RO_0002212 by negative regulation of teliospore formation [GO:0075258] Relationships: is a type of GO:0043936 Sources: GOC:pamgo_curators Definition: The set of processes leading to the formation of a thick-walled resting or over-wintering spore produced by the rust fungi (Uredinales) and smut fungi (Ustilaginales) in which karyogamy occurs.